3-aminomethylindole N-methyltransferase activity [GO:0102913] (molecular function) Definition: Catalysis of the reaction: 3-(aminomethyl)indole + S-adenosyl-L-methionine = (1H-indol-3-yl)-N-methylmethanamine + H+ + S-adenosyl-L-homocysteine. Relationships: is a type of GO:0008168 Sources: RHEA:52268